{
  "gene_name": "Atypical chemokine receptor 4",
  "term_id": "GO:0019722",
  "gene": "UniProtKB:Q9NPB9",
  "gene_symbol": "ACKR4",
  "term_label": "calcium-mediated signaling"
}